{
  "gene_symbol": "CLXN",
  "gene": "UniProtKB:Q9HAE3",
  "term_id": "GO:0005509",
  "gene_name": "Calaxin",
  "term_label": "calcium ion binding"
}